{
  "gene": "UniProtKB:Q30KQ6",
  "gene_symbol": "DEFB114",
  "term_label": "CCR6 chemokine receptor binding",
  "term_id": "GO:0031731",
  "gene_name": "Beta-defensin 114"
}